{
  "term_id": "GO:0000981",
  "gene_name": "LIM_homeobox protein Lhx3",
  "gene": "UniProtKB:Q9UBR4",
  "term_label": "DNA-binding transcription factor activity, RNA polymerase II-specific",
  "gene_symbol": "LHX3"
}